{
  "gene_symbol": "RNF43",
  "term_label": "Wnt receptor catabolic process",
  "term_id": "GO:0038018",
  "gene": "UniProtKB:Q68DV7",
  "gene_name": "E3 ubiquitin-protein ligase RNF43"
}